cell-cell adhesion involved in neural tube closure [GO:0060608] (BP) Relationships: is a type of GO:0060607; is part of neural tube closure [GO:0001843] Sources: GOC:dph Definition: The attachment of one cell to another cell along the edges of two epithelial folds, giving rise to the lumen of the neural tube. Subtypes: posterior neuropore closure [GO:0021507]